{
  "term_id": "GO:0051082",
  "gene_name": "Nascent polypeptide-associated complex subunit alpha, muscle-specific form",
  "gene": "UniProtKB:E9PAV3",
  "term_label": "unfolded protein binding",
  "gene_symbol": "NACA"
}